{
  "gene_name": "Pro-FMRFamide-related neuropeptide FF",
  "term_id": "GO:0005615",
  "term_label": "extracellular space",
  "gene": "UniProtKB:O15130",
  "gene_symbol": "NPFF"
}